sphingoid metabolic process [GO:0046519] (biological process) Sources: ISBN:0198506732 Relationships: is a type of sphingolipid metabolic process [GO:0006665] Definition: The chemical reactions and pathways involving sphingoids, any of a class of compounds comprising sphinganine and its homologues and stereoisomers, and derivatives of these compounds. Subtypes: 3-keto-sphinganine metabolic process [GO:0006666], sphinganine metabolic process [GO:0006667], sphingosine metabolic process [GO:0006670], phytosphingosine metabolic process [GO:0006671], sphingoid biosynthetic process [GO:0046520], sphingoid catabolic process [GO:0046521] Also known as: sphingoid base metabolic process, sphingoid base metabolism, sphingoid metabolism